positive regulation of triglyceride biosynthetic process [GO:0010867] (biological process) Sources: GOC:BHF, GOC:tb Definition: Any process that increases the rate, frequency, or extent of triglyceride biosynthesis. Triglyceride biosynthesis is the collection of chemical reactions and pathways resulting in the formation of triglyceride, any triester of glycerol. Relationships: is_a regulation of triglyceride biosynthetic process [GO:0010866]; is a type of positive regulation of lipid biosynthetic process [GO:0046889]; is a type of positive regulation of triglyceride metabolic process [GO:0090208]; positively regulates GO:0019432 Also known as: positive regulation of triacylglycerol biosynthetic process